{
  "gene_name": "Enoyl-CoA delta isomerase 2",
  "gene_symbol": "ECI2",
  "gene": "UniProtKB:O75521",
  "term_id": "GO:0005782",
  "term_label": "peroxisomal matrix"
}